{
  "gene": "UniProtKB:Q9NZM6",
  "gene_name": "Polycystin-2-like protein 2",
  "term_id": "GO:0050982",
  "term_label": "detection of mechanical stimulus",
  "gene_symbol": "PKD2L2"
}